{
  "gene": "UniProtKB:Q66K74",
  "term_label": "axonogenesis",
  "term_id": "GO:0007409",
  "gene_name": "Microtubule-associated protein 1S",
  "gene_symbol": "MAP1S"
}